{
  "gene": "UniProtKB:A0A1B0GVH7",
  "term_id": "UNKNOWN:0001",
  "gene_symbol": "IQCM",
  "gene_name": "IQ domain-containing protein M",
  "term_label": "Unknown molecular function"
}